{
  "term_label": "plasma membrane",
  "gene_symbol": "LSAMP",
  "gene_name": "Limbic system-associated membrane protein",
  "term_id": "GO:0005886",
  "gene": "UniProtKB:Q13449"
}